{
  "term_id": "UNKNOWN:0002",
  "gene_name": "Ovostatin homolog 1",
  "gene": "UniProtKB:Q6IE37",
  "gene_symbol": "OVOS1",
  "term_label": "Unknown biological process"
}